{
  "gene_name": "Protein kinase C-binding protein NELL1",
  "gene": "UniProtKB:Q92832",
  "gene_symbol": "NELL1",
  "term_label": "positive regulation of ossification",
  "term_id": "GO:0045778"
}